{
  "gene": "UniProtKB:Q92539",
  "gene_symbol": "LPIN2",
  "gene_name": "Phosphatidate phosphatase LPIN2",
  "term_label": "fatty acid catabolic process",
  "term_id": "GO:0009062"
}